{
  "gene": "UniProtKB:Q9UHA4",
  "gene_name": "Ragulator complex protein LAMTOR3",
  "gene_symbol": "LAMTOR3",
  "term_id": "GO:0071986",
  "term_label": "Ragulator complex"
}